{
  "gene_name": "Transmembrane protein 39A",
  "gene_symbol": "TMEM39A",
  "gene": "UniProtKB:Q9NV64",
  "term_label": "negative regulation of autophagosome maturation",
  "term_id": "GO:1901097"
}